{
  "term_id": "GO:0005096",
  "gene": "UniProtKB:Q6ZUM4",
  "gene_name": "Rho GTPase-activating protein 27",
  "gene_symbol": "ARHGAP27",
  "term_label": "GTPase activator activity"
}